ethylene binding [GO:0051740] (molecular function) Relationships: is a type of alkene binding [GO:0072328] Also known as: ethene binding Sources: GOC:ai Definition: Binding to ethylene (C2-H4, ethene), a simple hydrocarbon gas that can function in plants as a growth regulator.